modulation of chemical synaptic transmission [GO:0050804] (biological process) Definition: Any process that modulates the frequency or amplitude of synaptic transmission, the process of communication from a neuron to a target (neuron, muscle, or secretory cell) across a synapse. Amplitude, in this case, refers to the change in postsynaptic membrane potential due to a single instance of synaptic transmission. Sources: GOC:ai Also known as: modulation of synaptic transmission, regulation of chemical synaptic transmission, regulation of synaptic transmission Relationships: is a type of regulation of trans-synaptic signaling [GO:0099177]; regulates chemical synaptic transmission [GO:0007268] Subtypes: regulation of synaptic transmission, cholinergic [GO:0032222], GO:0032225, regulation of synaptic transmission, GABAergic [GO:0032228], regulation of neurotransmitter secretion [GO:0046928], regulation of synaptic plasticity [GO:0048167], negative regulation of synaptic transmission [GO:0050805], GO:0050806, regulation of synaptic transmission, glutamatergic [GO:0051966], GO:0060024, regulation of synaptic activity [GO:0060025], regulation of synaptic transmission, glycinergic [GO:0060092], GO:0098815, GO:0098987, postsynaptic modulation of chemical synaptic transmission [GO:0099170], GO:0099171, regulation of translation at synapse, modulating synaptic transmission [GO:0099547], trans-synaptic signaling, modulating synaptic transmission [GO:0099550], GO:0099574, regulation of spontaneous synaptic transmission [GO:0150003], GO:0150035, regulation of trans-synaptic signaling by endocannabinoid, modulating synaptic transmission [GO:0150036], regulation of neuromuscular synaptic transmission [GO:1900073]